{
  "term_label": "innate immune response",
  "gene_symbol": "RNASE8",
  "gene_name": "Ribonuclease 8",
  "gene": "UniProtKB:Q8TDE3",
  "term_id": "GO:0045087"
}